positive regulation of helvolic acid biosynthetic process [GO:1900842] (biological process) Also known as: up regulation of helvolic acid biosynthetic process, up-regulation of helvolic acid biosynthetic process, upregulation of helvolic acid biosynthetic process Sources: GOC:TermGenie, GOC:di Definition: Any process that activates or increases the frequency, rate or extent of helvolic acid biosynthetic process. Relationships: is_a GO:0010893; is a type of positive regulation of small molecule metabolic process [GO:0062013]; is a type of GO:1900378; is a type of regulation of helvolic acid biosynthetic process [GO:1900840]; positively regulates GO:1900812